{
  "gene_symbol": "ZNF335",
  "gene_name": "Zinc finger protein 335",
  "term_id": "GO:0003700",
  "term_label": "DNA-binding transcription factor activity",
  "gene": "UniProtKB:Q9H4Z2"
}